metanephric juxtaglomerulus cell development [GO:0072252] (biological process) Definition: The process whose specific outcome is the progression of a metanephric juxtaglomerulus cell over time, from its formation to the mature structure. Relationships: is a type of GO:0072142; is part of GO:0072251 Sources: GOC:mtg_kidney_jan10